{
  "gene_name": "Lysosome membrane protein 2",
  "term_label": "lysosomal membrane",
  "gene_symbol": "SCARB2",
  "term_id": "GO:0005765",
  "gene": "UniProtKB:Q14108"
}